{
  "gene": "UniProtKB:P57735",
  "gene_name": "Ras-related protein Rab-25",
  "term_id": "GO:0005794",
  "gene_symbol": "RAB25",
  "term_label": "Golgi apparatus"
}